{
  "gene_name": "HLA class II histocompatibility antigen, DQ alpha 2 chain",
  "term_id": "GO:0050870",
  "gene_symbol": "HLA-DQA2",
  "gene": "UniProtKB:P01906",
  "term_label": "positive regulation of T cell activation"
}